{
  "gene_symbol": "C19orf81",
  "term_label": "Unknown cellular component",
  "gene": "UniProtKB:C9J6K1",
  "gene_name": "Putative uncharacterized protein C19orf81",
  "term_id": "UNKNOWN:0003"
}